{
  "term_label": "cytoplasm",
  "term_id": "GO:0005737",
  "gene": "UniProtKB:P31947",
  "gene_symbol": "SFN",
  "gene_name": "14-3-3 protein sigma"
}